{
  "gene_symbol": "XRCC4",
  "term_label": "immunoglobulin V(D)J recombination",
  "gene": "UniProtKB:Q13426",
  "term_id": "GO:0033152",
  "gene_name": "DNA repair protein XRCC4"
}